{
  "term_id": "GO:1903706",
  "term_label": "regulation of hemopoiesis",
  "gene_name": "Zinc finger protein Gfi-1b",
  "gene": "UniProtKB:Q5VTD9",
  "gene_symbol": "GFI1B"
}